{
  "term_label": "Unknown cellular component",
  "gene": "UniProtKB:Q8NCT3",
  "gene_name": "Putative tyrosine carboxypeptidase MATCAP2",
  "term_id": "UNKNOWN:0003",
  "gene_symbol": "MATCAP2"
}